{
  "gene": "UniProtKB:Q5VYP0",
  "gene_name": "Spermatogenesis-associated protein 31A3",
  "term_label": "Unknown cellular component",
  "term_id": "UNKNOWN:0003",
  "gene_symbol": "SPATA31A3"
}